detection of molecule of oomycetes origin [GO:0032492] (biological process) Sources: GOC:mah, GOC:rl Definition: The series of events in which a stimulus from a molecule of oomycetes origin is received and converted into a molecular signal. Also known as: detection of oomycetes associated molecule Relationships: is a type of response to molecule of oomycetes origin [GO:0002240]; is a type of GO:0009593; is a type of detection of external biotic stimulus [GO:0098581]